{
  "term_label": "plasma membrane",
  "gene_symbol": "PLXNA3",
  "term_id": "GO:0005886",
  "gene": "UniProtKB:P51805",
  "gene_name": "Plexin-A3"
}